{
  "gene": "UniProtKB:Q92949",
  "term_id": "GO:0000978",
  "gene_name": "Forkhead box protein J1",
  "term_label": "RNA polymerase II cis-regulatory region sequence-specific DNA binding",
  "gene_symbol": "FOXJ1"
}